{
  "term_label": "Unknown molecular function",
  "term_id": "UNKNOWN:0001",
  "gene_symbol": "MARCHF10",
  "gene": "UniProtKB:Q8NA82",
  "gene_name": "Probable E3 ubiquitin-protein ligase MARCHF10"
}